protection from natural killer cell mediated cytotoxicity [GO:0042270] (biological process) Also known as: protection from NK cell mediated cell death, protection from NK cell mediated cell killing, protection from NK cell mediated cytotoxicity, protection from natural killer cell mediated cell death, protection from natural killer cell mediated cell killing, protection from NK cell mediated cytolysis, protection from natural killer cell mediated cytolysis Relationships: is a type of negative regulation of natural killer cell mediated cytotoxicity [GO:0045953] Sources: GOC:add, ISBN:0781735149 Definition: The process of protecting a cell from natural killer cell mediated cytotoxicity.